regulation of epithelium regeneration [GO:1905041] (biological process) Also known as: regulation of regeneration of epithelium Relationships: is a type of GO:0048638; regulates GO:1990399 References: PMID:23221517 Sources: GOC:BHF, GOC:BHF_miRNA, GOC:TermGenie, GOC:rph, GO_REF:0000058 Definition: Any process that modulates the frequency, rate or extent of epithelium regeneration. Subtypes: negative regulation of epithelium regeneration [GO:1905042], positive regulation of epithelium regeneration [GO:1905043]